IgM receptor activity [GO:0001793] (molecular function) Definition: Combining with an immunoglobulin of the IgM isotype via the Fc region, and transmitting the signal from one side of the membrane to the other to initiate a change in cell activity. Sources: GOC:add, GOC:signaling, ISBN:0781735149 Subtypes: high-affinity IgM receptor activity [GO:0002172], low-affinity IgM receptor activity [GO:0002173] Relationships: is a type of GO:0019763; has part IgM binding [GO:0001791]